{
  "gene": "UniProtKB:A0A191URJ7",
  "term_label": "immune receptor activity",
  "gene_symbol": "KIR2DL1",
  "term_id": "GO:0140375",
  "gene_name": "KIR2DL protein"
}